{
  "gene": "UniProtKB:Q9UJV9",
  "gene_symbol": "DDX41",
  "term_id": "GO:0000398",
  "gene_name": "Probable ATP-dependent RNA helicase DDX41",
  "term_label": "mRNA splicing, via spliceosome"
}